{
  "term_id": "GO:0070098",
  "term_label": "chemokine-mediated signaling pathway",
  "gene": "UniProtKB:P13236",
  "gene_symbol": "CCL4",
  "gene_name": "C-C motif chemokine 4"
}